{
  "gene": "UniProtKB:P50443",
  "gene_name": "Sulfate transporter",
  "term_label": "oxalate transmembrane transporter activity",
  "gene_symbol": "SLC26A2",
  "term_id": "GO:0019531"
}